regulation of asymmetric protein localization involved in cell fate determination [GO:1904785] (biological process) Subtypes: negative regulation of asymmetric protein localization involved in cell fate determination [GO:1904786], positive regulation of asymmetric protein localization involved in cell fate determination [GO:1904787] Definition: Any process that modulates the frequency, rate or extent of asymmetric protein localization involved in cell fate determination. References: PMID:17476329 Sources: GOC:TermGenie, GO_REF:0000058 Relationships: is a type of regulation of protein localization [GO:0032880]; is a type of regulation of cell fate determination [GO:1905933]; regulates asymmetric protein localization involved in cell fate determination [GO:0045167] Note: wrm-1 in C. Elegans (Q10953) in PMID:17476329 (IMP) Also known as: regulation of asymmetric protein localisation involved in cell fate determination, regulation of asymmetric protein localization involved in cell fate commitment, regulation of asymmetric protein localization resulting in cell fate commitment, regulation of cell fate commitment, asymmetric protein localization